IgD immunoglobulin complex, circulating [GO:0071739] (cellular component) Also known as: IgD antibody References: PMID:11282392 Sources: GOC:add, ISBN:0781765196 Definition: A protein complex composed of two identical immunoglobulin heavy chains of the IgD isotype and two identical immunoglobulin light chains, held together by disulfide bonds, and present in the extracellular space, in mucosal areas or other tissues, or circulating in the blood or lymph. Note: Note that an IgD immunoglobulin complex has the function of antigen binding if a suitable antigen is available. Relationships: is a type of immunoglobulin complex, circulating [GO:0042571]; is a type of GO:0071738